grooming behavior [GO:0007625] (biological process) Sources: GOC:jl, GOC:pr Relationships: is a type of behavior [GO:0007610] Also known as: grooming behaviour Regulation: regulated by GO:2000821 Definition: The specific behavior of an organism relating to grooming, cleaning and brushing to remove dirt and parasites.